{
  "gene_symbol": "TMEM121",
  "term_label": "Unknown cellular component",
  "term_id": "UNKNOWN:0003",
  "gene_name": "Transmembrane protein 121",
  "gene": "UniProtKB:Q9BTD3"
}